{
  "gene": "UniProtKB:Q9UGF5",
  "term_id": "GO:0004984",
  "gene_name": "Olfactory receptor 14J1",
  "term_label": "olfactory receptor activity",
  "gene_symbol": "OR14J1"
}